{
  "gene_name": "Homeobox protein GBX-2",
  "gene_symbol": "GBX2",
  "gene": "UniProtKB:P52951",
  "term_label": "nucleus",
  "term_id": "GO:0005634"
}